ADP transport [GO:0015866] (biological process) Subtypes: mitochondrial ADP transmembrane transport [GO:0140021] Sources: GOC:ai Definition: The directed movement of ADP, adenosine diphosphate, into, out of or within a cell, or between cells, by means of some agent such as a transporter or pore. Relationships: is_a organic anion transport [GO:0015711]; is a type of purine ribonucleotide transport [GO:0015868]; is a type of GO:0051503